{
  "gene": "UniProtKB:Q1MX18",
  "gene_symbol": "INSC",
  "term_label": "apical cortex",
  "gene_name": "Protein inscuteable homolog",
  "term_id": "GO:0045179"
}